galactose:sodium symporter activity [GO:0015371] (molecular function) Definition: Enables the transfer of a solute or solutes from one side of a membrane to the other according to the reaction: galactose(out) + Na+(out) = glucose(in) + Na+(in). Relationships: is a type of GO:0005354; is a type of carbohydrate:monoatomic cation symporter activity [GO:0005402]; is a type of solute:sodium symporter activity [GO:0015370] Sources: TC:2.A.21.3.-